{
  "term_label": "membrane",
  "gene": "UniProtKB:P0CG39",
  "term_id": "GO:0016020",
  "gene_name": "POTE ankyrin domain family member J",
  "gene_symbol": "POTEJ"
}